{
  "gene_name": "Tyrosine-protein kinase receptor TYRO3",
  "gene_symbol": "TYRO3",
  "gene": "UniProtKB:Q06418",
  "term_id": "GO:0005886",
  "term_label": "plasma membrane"
}